{
  "gene_name": "Platelet-derived growth factor subunit A",
  "gene_symbol": "PDGFA",
  "gene": "UniProtKB:P04085",
  "term_label": "platelet-derived growth factor receptor signaling pathway",
  "term_id": "GO:0048008"
}